negative regulation of endothelial cell differentiation [GO:0045602] (biological process) Also known as: down regulation of endothelial cell differentiation, down-regulation of endothelial cell differentiation, downregulation of endothelial cell differentiation, inhibition of endothelial cell differentiation Sources: GOC:go_curators Definition: Any process that stops, prevents, or reduces the frequency, rate or extent of endothelial cell differentiation. Relationships: is a type of negative regulation of epithelial cell differentiation [GO:0030857]; is a type of GO:0045601; RO_0002212 GO:0045446 Subtypes: negative regulation of blood vessel endothelial cell differentiation [GO:0110059], negative regulation of endothelial cell development [GO:1901551]